pyloric canal smooth muscle contraction [GO:0120066] (biological process) Relationships: is_a stomach pylorus smooth muscle contraction [GO:0120064] Definition: A process in which force is generated within gastric smooth muscle tissue, resulting in a change in muscle geometry. This process occurs in the distal part of the pylorus between the pyloric antrum and the pyloric sphincter. References: PMID:15890336 Sources: GOC:sl